{
  "gene_symbol": "CD8A",
  "term_label": "cell surface receptor signaling pathway",
  "gene_name": "T-cell surface glycoprotein CD8 alpha chain",
  "term_id": "GO:0007166",
  "gene": "UniProtKB:P01732"
}